smoothened signaling pathway involved in dorsal/ventral neural tube patterning [GO:0060831] (biological process) Relationships: is a type of smoothened signaling pathway [GO:0007224]; is part of dorsal/ventral neural tube patterning [GO:0021904] Also known as: hedgehog signaling pathway involved in dorsal/ventral neural tube patterning, hh signaling pathway involved in dorsal/ventral neural tube patterning, smoothened signalling pathway involved in dorsal/ventral neural tube patterning Definition: The series of molecular signals generated as a consequence of activation of the transmembrane protein Smoothened contributing to the dorsal/ventral pattern of the neural tube. Sources: GOC:dph, GOC:sdb_2009, GOC:tb Regulation: regulated by GO:1901620; negatively regulated by negative regulation of smoothened signaling pathway involved in dorsal/ventral neural tube patterning [GO:1901621]; positively regulated by positive regulation of smoothened signaling pathway involved in dorsal/ventral neural tube patterning [GO:1901622]